{
  "gene_name": "Synembryn-B",
  "gene": "UniProtKB:Q9NVN3",
  "gene_symbol": "RIC8B",
  "term_label": "cytoplasm",
  "term_id": "GO:0005737"
}